{
  "gene": "UniProtKB:Q5U651",
  "gene_symbol": "RASIP1",
  "gene_name": "Ras-interacting protein 1",
  "term_id": "GO:0001525",
  "term_label": "angiogenesis"
}